{
  "gene_symbol": "SERP2",
  "term_id": "GO:0030968",
  "term_label": "endoplasmic reticulum unfolded protein response",
  "gene_name": "Stress-associated endoplasmic reticulum protein 2",
  "gene": "UniProtKB:Q8N6R1"
}